{
  "gene_symbol": "NR0B2",
  "gene": "UniProtKB:Q15466",
  "gene_name": "Nuclear receptor subfamily 0 group B member 2",
  "term_label": "nucleus",
  "term_id": "GO:0005634"
}